{
  "gene": "UniProtKB:A0A2U3TZM8",
  "term_id": "UNKNOWN:0001",
  "gene_symbol": "LOC112694756",
  "gene_name": "Uncharacterized protein",
  "term_label": "Unknown molecular function"
}